{
  "term_label": "regulation of transcription by RNA polymerase II",
  "gene_symbol": "ZHX3",
  "term_id": "GO:0006357",
  "gene": "UniProtKB:Q9H4I2",
  "gene_name": "Zinc fingers and homeoboxes protein 3"
}